{
  "term_label": "Unknown cellular component",
  "gene_symbol": "ZSWIM2",
  "gene_name": "E3 ubiquitin-protein ligase ZSWIM2",
  "gene": "UniProtKB:Q8NEG5",
  "term_id": "UNKNOWN:0003"
}